{
  "gene": "UniProtKB:P08134",
  "term_id": "GO:0032956",
  "term_label": "regulation of actin cytoskeleton organization",
  "gene_name": "Rho-related GTP-binding protein RhoC",
  "gene_symbol": "RHOC"
}